{
  "gene_symbol": "CENPV",
  "term_id": "GO:0032467",
  "term_label": "positive regulation of cytokinesis",
  "gene_name": "Centromere protein V",
  "gene": "UniProtKB:Q7Z7K6"
}